{
  "gene": "UniProtKB:Q9BX63",
  "term_id": "GO:1990918",
  "gene_symbol": "BRIP1",
  "term_label": "double-strand break repair involved in meiotic recombination",
  "gene_name": "Fanconi anemia group J protein"
}